peroxidase activity [GO:0004601] (molecular function) Sources: GOC:curators Regulation: negatively regulated by peroxidase inhibitor activity [GO:0036479] Relationships: is a type of antioxidant activity [GO:0016209]; is a type of oxidoreductase activity, acting on peroxide as acceptor [GO:0016684] Definition: Catalysis of the reaction: a donor + a peroxide = an oxidized donor + 2 H2O. Subtypes: catalase activity [GO:0004096], cytochrome-c peroxidase activity [GO:0004130], GO:0004602, L-ascorbate peroxidase activity [GO:0016688], GO:0016689, diarylpropane peroxidase activity [GO:0016690], NADH peroxidase activity [GO:0016692], tryparedoxin peroxidase activity [GO:0033196], thiocyanate peroxidase activity [GO:0036393], phospholipid-hydroperoxide glutathione peroxidase activity [GO:0047066], fatty acid peroxidase activity [GO:0047888], NADPH peroxidase activity [GO:0050137], peroxiredoxin activity [GO:0051920], GO:0052750, GO:0072541, lactoperoxidase activity [GO:0140825], haloperoxidase activity [GO:0140905] Also known as: peroxidase reaction, bacterial catalase-peroxidase activity, eosinophil peroxidase activity, extensin peroxidase, guaiacol peroxidase, heme peroxidase, horseradish peroxidase (HRP), japanese radish peroxidase, lactoperoxidase activity, myeloperoxidase activity, protoheme peroxidase, pyrocatechol peroxidase, scopoletin peroxidase, secretory plant peroxidase activity, thiocyanate peroxidase, verdoperoxidase, MPO, donor:hydrogen-peroxide oxidoreductase activity, oxyperoxidase activity